{
  "gene": "UniProtKB:Q96MP8",
  "gene_symbol": "KCTD7",
  "gene_name": "BTB_POZ domain-containing protein KCTD7",
  "term_label": "membrane hyperpolarization",
  "term_id": "GO:0060081"
}